{
  "term_id": "GO:0022858",
  "term_label": "alanine transmembrane transporter activity",
  "gene": "UniProtKB:Q9UN76",
  "gene_name": "Sodium- and chloride-dependent neutral and basic amino acid transporter B(0+)",
  "gene_symbol": "SLC6A14"
}